cibarial fish-trap bristle development [GO:0048725] (biological process) Relationships: is a type of GO:0022416; is part of clypeo-labral disc development [GO:0035213] Also known as: fish-trap bristle development Sources: FBbt:00004136, GOC:rc Definition: The process whose specific outcome is the progression of the cibarial fish-trap bristle over time, from its formation to the mature structure. A cibarial fish-trap bristle is a sensory bristle on the anterior plate of the cibarium.